positive regulation of lipase activity [GO:0060193] (biological process) Relationships: is a type of positive regulation of hydrolase activity [GO:0051345]; positively regulates lipase activity [GO:0016298] Subtypes: positive regulation of phospholipase activity [GO:0010518], positive regulation of triglyceride lipase activity [GO:0061365] Sources: GOC:BHF, GOC:dph, GOC:tb Definition: Any process that increases the frequency, rate or extent of lipase activity, the hydrolysis of a lipid or phospholipid.